{
  "gene": "UniProtKB:Q5VYJ5",
  "gene_name": "MAM and LDL-receptor class A domain-containing protein 1",
  "gene_symbol": "MALRD1",
  "term_id": "UNKNOWN:0001",
  "term_label": "Unknown molecular function"
}